{
  "gene_name": "Beta-2-microglobulin",
  "gene": "UniProtKB:P61769",
  "term_id": "GO:0005765",
  "term_label": "lysosomal membrane",
  "gene_symbol": "B2M"
}